{
  "gene_name": "Interleukin-18",
  "gene": "UniProtKB:Q14116",
  "gene_symbol": "IL18",
  "term_label": "cytokine-mediated signaling pathway",
  "term_id": "GO:0019221"
}